{
  "gene": "UniProtKB:Q9Y248",
  "term_label": "GINS complex",
  "gene_name": "DNA replication complex GINS protein PSF2",
  "gene_symbol": "GINS2",
  "term_id": "GO:0000811"
}